{
  "gene_symbol": "NR3C1",
  "gene": "UniProtKB:P04150",
  "gene_name": "Glucocorticoid receptor",
  "term_id": "GO:0004879",
  "term_label": "nuclear receptor activity"
}